{
  "gene": "UniProtKB:Q9H1A4",
  "term_id": "GO:0060090",
  "gene_symbol": "ANAPC1",
  "term_label": "molecular adaptor activity",
  "gene_name": "Anaphase-promoting complex subunit 1"
}